{
  "gene": "UniProtKB:Q92499",
  "gene_symbol": "DDX1",
  "gene_name": "ATP-dependent RNA helicase DDX1",
  "term_label": "Unknown molecular function",
  "term_id": "UNKNOWN:0001"
}